{
  "term_id": "GO:0003735",
  "term_label": "structural constituent of ribosome",
  "gene_symbol": "RPL19",
  "gene_name": "Large ribosomal subunit protein eL19",
  "gene": "UniProtKB:P84098"
}